positive regulation of synaptic vesicle fusion to presynaptic active zone membrane [GO:0031632] (biological process) Definition: Any process that activates or increases the frequency, rate or extent of synaptic vesicle fusion to the presynaptic membrane. Sources: GOC:mah Relationships: is a type of positive regulation of vesicle fusion [GO:0031340]; is a type of regulation of synaptic vesicle fusion to presynaptic active zone membrane [GO:0031630]; is_a positive regulation of synaptic vesicle membrane organization [GO:1901634]; positively regulates synaptic vesicle fusion to presynaptic active zone membrane [GO:0031629] Subtypes: calcium-dependent activation of synaptic vesicle fusion [GO:0099502] Also known as: negative regulation of synaptic vesicle fusion to presynaptic membrane, positive regulation of synaptic vesicle fusion to pre-synaptic membrane, up regulation of synaptic vesicle fusion to presynaptic active zone membrane, up regulation of synaptic vesicle fusion to presynaptic membrane, up-regulation of synaptic vesicle fusion to presynaptic active zone membrane, up-regulation of synaptic vesicle fusion to presynaptic membrane, upregulation of synaptic vesicle fusion to presynaptic membrane, activation of synaptic vesicle fusion to presynaptic membrane, stimulation of synaptic vesicle fusion to presynaptic membrane